{
  "term_id": "GO:0004674",
  "gene_name": "Bromodomain-containing protein 4",
  "term_label": "protein serine/threonine kinase activity",
  "gene_symbol": "BRD4",
  "gene": "UniProtKB:O60885"
}